{
  "term_label": "smooth muscle cell migration",
  "gene_symbol": "PLAT",
  "term_id": "GO:0014909",
  "gene": "UniProtKB:P00750",
  "gene_name": "Tissue-type plasminogen activator"
}